{
  "term_label": "Unknown molecular function",
  "gene": "UniProtKB:Q8NA75",
  "gene_name": "DDB1- and CUL4-associated factor 4-like protein 2",
  "term_id": "UNKNOWN:0001",
  "gene_symbol": "DCAF4L2"
}